{
  "gene_name": "Transcription factor SOX-12",
  "gene_symbol": "SOX12",
  "gene": "UniProtKB:O15370",
  "term_id": "GO:0048593",
  "term_label": "camera-type eye morphogenesis"
}